beta-acoradiene synthase activity [GO:0102882] (molecular function) Definition: Catalysis of the reaction: (2E,6E)-farnesyl diphosphate = beta-acoradiene + diphosphate. Sources: RHEA:68520 Relationships: is a type of carbon-oxygen lyase activity, acting on phosphates [GO:0016838]